{
  "gene": "UniProtKB:Q7L5N7",
  "term_id": "UNKNOWN:0002",
  "term_label": "Unknown biological process",
  "gene_name": "Lysophosphatidylcholine acyltransferase 2",
  "gene_symbol": "LPCAT2"
}